negative regulation of cholangiocyte apoptotic process [GO:1904193] (biological process) Relationships: is a type of negative regulation of epithelial cell apoptotic process [GO:1904036]; is_a regulation of cholangiocyte apoptotic process [GO:1904192]; negatively regulates GO:1902488 Also known as: down regulation of cholangiocyte apoptotic process, down regulation of epithelial cell of bile duct apoptotic process, down-regulation of cholangiocyte apoptotic process, down-regulation of epithelial cell of bile duct apoptotic process, downregulation of cholangiocyte apoptotic process, downregulation of epithelial cell of bile duct apoptotic process, negative regulation of epithelial cell of bile duct apoptotic process, down regulation of cholangiocyte apoptosis, down regulation of epithelial cell of bile duct apoptosis, down-regulation of cholangiocyte apoptosis, down-regulation of epithelial cell of bile duct apoptosis, downregulation of cholangiocyte apoptosis, downregulation of epithelial cell of bile duct apoptosis, inhibition of cholangiocyte apoptosis, inhibition of cholangiocyte apoptotic process, inhibition of epithelial cell of bile duct apoptosis, inhibition of epithelial cell of bile duct apoptotic process, negative regulation of cholangiocyte apoptosis, negative regulation of epithelial cell of bile duct apoptosis Definition: Any process that stops, prevents or reduces the frequency, rate or extent of cholangiocyte apoptotic process. References: PMID:24498161 Sources: GOC:TermGenie, GO_REF:0000058